{
  "term_id": "GO:0016477",
  "gene": "UniProtKB:O43281",
  "gene_name": "Embryonal Fyn-associated substrate",
  "term_label": "cell migration",
  "gene_symbol": "EFS"
}